{
  "term_label": "RNA polymerase II cis-regulatory region sequence-specific DNA binding",
  "gene_symbol": "ZNF420",
  "gene_name": "Zinc finger protein 420",
  "term_id": "GO:0000978",
  "gene": "UniProtKB:Q8TAQ5"
}